{
  "gene": "UniProtKB:Q6V0L0",
  "term_label": "Unknown cellular component",
  "gene_symbol": "CYP26C1",
  "term_id": "UNKNOWN:0003",
  "gene_name": "Cytochrome P450 26C1"
}